phosphocholine transferase activity [GO:0044605] (MF) References: PMID:21822290 Sources: GOC:sp Relationships: is a type of phosphotransferase activity, alcohol group as acceptor [GO:0016773] Definition: Catalysis of the reaction: CDP-choline + protein-serine = CMP + protein-serine-choline phosphate.